{
  "term_label": "Unknown biological process",
  "gene_name": "G-protein coupled receptor family C group 5 member D",
  "gene": "UniProtKB:Q9NZD1",
  "gene_symbol": "GPRC5D",
  "term_id": "UNKNOWN:0002"
}